{
  "gene": "UniProtKB:Q9Y6N7",
  "term_id": "UNKNOWN:0001",
  "term_label": "Unknown molecular function",
  "gene_name": "Roundabout homolog 1",
  "gene_symbol": "ROBO1"
}